{
  "gene_name": "Kallikrein-2",
  "term_label": "zymogen activation",
  "term_id": "GO:0031638",
  "gene": "UniProtKB:P20151",
  "gene_symbol": "KLK2"
}